late endosome lumen [GO:0031906] (CC) Definition: The volume enclosed by the membrane of a late endosome. Sources: GOC:mah Relationships: is a type of endosome lumen [GO:0031904]; BFO_0000050 late endosome [GO:0005770] Subtypes: GO:0097486